{
  "gene_symbol": "PLCD1",
  "term_id": "GO:0004435",
  "gene_name": "1-phosphatidylinositol 4,5-bisphosphate phosphodiesterase delta-1",
  "gene": "UniProtKB:P51178",
  "term_label": "phosphatidylinositol-4,5-bisphosphate phospholipase C activity"
}